{
  "term_id": "GO:0000978",
  "gene_name": "Zinc finger protein 121",
  "term_label": "RNA polymerase II cis-regulatory region sequence-specific DNA binding",
  "gene": "UniProtKB:P58317",
  "gene_symbol": "ZNF121"
}